{
  "term_id": "UNKNOWN:0001",
  "gene": "UniProtKB:P0DMW3",
  "gene_name": "Small integral membrane protein 10-like protein 1",
  "gene_symbol": "SMIM10L1",
  "term_label": "Unknown molecular function"
}